{
  "gene_symbol": "TNP1",
  "term_id": "GO:0003677",
  "gene_name": "Spermatid nuclear transition protein 1",
  "gene": "UniProtKB:P09430",
  "term_label": "DNA binding"
}